{
  "gene_symbol": "OR5D18",
  "term_label": "G protein-coupled receptor signaling pathway",
  "gene_name": "Olfactory receptor 5D18",
  "gene": "UniProtKB:Q8NGL1",
  "term_id": "GO:0007186"
}